{
  "term_id": "GO:0006833",
  "gene_name": "Aquaporin-2",
  "gene_symbol": "AQP2",
  "term_label": "water transport",
  "gene": "UniProtKB:P41181"
}